{
  "gene": "UniProtKB:Q9ULB1",
  "term_label": "adult behavior",
  "gene_name": "Neurexin-1",
  "gene_symbol": "NRXN1",
  "term_id": "GO:0030534"
}